{
  "gene": "UniProtKB:A0A0A0MRZ9",
  "term_id": "GO:0006955",
  "term_label": "immune response",
  "gene_name": "Immunoglobulin lambda variable 5-52",
  "gene_symbol": "IGLV5-52"
}